benzoate 1,2-dioxygenase activity [GO:0018623] (molecular function) Also known as: benzoate dioxygenase activity, benzoate hydroxylase activity, benzoate,NADH:oxygen oxidoreductase (1,2-hydroxylating), benzoate,NADH:oxygen oxidoreductase (1,2-hydroxylating, decarboxylating), benzoic hydroxylase activity Definition: Catalysis of the reaction: benzoate + NADH + H+ + O2 = catechol + CO2 + NAD+. Sources: EC:1.14.12.10 Relationships: is a type of oxidoreductase activity, acting on paired donors, with incorporation or reduction of molecular oxygen, NAD(P)H as one donor, and incorporation of two atoms of oxygen into one donor [GO:0016708]